box H/ACA snoRNP assembly [GO:0000493] (BP) Also known as: box H/ACA small nucleolar ribonucleoprotein complex assembly References: PMID:12515383 Sources: GOC:krc Definition: The aggregation, arrangement and bonding together of proteins and a box H/ACA snoRNA to form a box H/ACA small nucleolar ribonucleoprotein (snoRNP) complex. Relationships: is a type of GO:0000491